oxidoreductase complex [GO:1990204] (cellular component) Relationships: is a type of GO:1902494 References: PMID:18982432 Sources: GOC:bhm Definition: Any protein complex that possesses oxidoreductase activity. Subtypes: 5-lipoxygenase complex [GO:0002180], xanthine dehydrogenase complex [GO:0002197], GO:0005960, ribonucleoside-diphosphate reductase complex [GO:0005971], cytochrome o ubiquinol oxidase complex [GO:0009319], GO:0009324, nitrate reductase complex [GO:0009325], GO:0009326, GO:0009331, 3-phenylpropionate dioxygenase complex [GO:0009334], glycolate oxidase complex [GO:0009339], ferredoxin hydrogenase complex [GO:0009375], photosystem II oxygen evolving complex [GO:0009654], methane monooxygenase complex [GO:0015050], procollagen-proline 4-dioxygenase complex [GO:0016222], nitrogenase complex [GO:0016610], ferredoxin-thioredoxin reductase complex [GO:0030386], glycine reductase complex [GO:0030700], GO:0030964, glutamate synthase complex [GO:0031026], sarcosine oxidase complex [GO:0032921], fatty acid beta-oxidation multienzyme complex [GO:0036125], NADPH oxidase complex [GO:0043020], GO:0044678, methanophenazine reducing hydrogenase complex [GO:0044679], alpha-ketoacid dehydrogenase complex [GO:0045240], isocitrate dehydrogenase complex (NAD+) [GO:0045242], respiratory chain complex II (succinate dehydrogenase) [GO:0045273], phenylacetyl-CoA 1,2-epoxidase complex [GO:0062077], catalase complex [GO:0062151], dihydropyrimidine dehydrogenase (NAD+) complex [GO:0140690], thioredoxin-disulfide reductase complex [GO:1902515], GO:1902560, superoxide dismutase complex [GO:1902693], pyrroline-5-carboxylate reductase complex [GO:1902792], GO:1903958, trimethylamine-N-oxide reductase (cytochrome c) complex [GO:1904852], ferroxidase complex [GO:1905862], glutamate dehydrogenase complex [GO:1990148], alkanesulfonate monooxygenase complex [GO:1990201], FMN reductase complex [GO:1990202], taurine dioxygenase complex [GO:1990205] Also known as: oxidation-reduction complex, redox complex